{
  "term_label": "inflammatory response",
  "gene_symbol": "CCR2",
  "gene_name": "C-C chemokine receptor type 2",
  "term_id": "GO:0006954",
  "gene": "UniProtKB:P41597"
}